{
  "term_id": "GO:0001517",
  "gene": "UniProtKB:Q7LGC8",
  "gene_symbol": "CHST3",
  "term_label": "N-acetylglucosamine 6-O-sulfotransferase activity",
  "gene_name": "Carbohydrate sulfotransferase 3"
}